{
  "gene": "UniProtKB:Q96BT7",
  "gene_name": "Alkylated DNA repair protein alkB homolog 8",
  "gene_symbol": "ALKBH8",
  "term_id": "GO:0005737",
  "term_label": "cytoplasm"
}